{
  "term_label": "alpha-mannosidase activity",
  "term_id": "GO:0004559",
  "gene_symbol": "MANEAL",
  "gene": "UniProtKB:Q5VSG8",
  "gene_name": "Glycoprotein endo-alpha-1,2-mannosidase-like protein"
}